auxin export across the plasma membrane [GO:0010315] (biological process) Definition: The directed movement of auxins from inside of a cell, across the plasma membrane and into the extracellular region. Relationships: is_a GO:0010928; is a type of auxin transport [GO:0060918]; is_a export across plasma membrane [GO:0140115] References: PMID:16990790 Sources: GOC:tair_curators Also known as: auxin efflux, auxin export